{
  "term_label": "cytokine receptor activity",
  "gene_name": "Oncostatin-M-specific receptor subunit beta",
  "gene": "UniProtKB:Q99650",
  "term_id": "GO:0004896",
  "gene_symbol": "OSMR"
}